{
  "gene_name": "Ig-like domain-containing protein (Fragment)",
  "gene_symbol": "A0A0J9YWU9",
  "gene": "UniProtKB:A0A0J9YWU9",
  "term_label": "Unknown cellular component",
  "term_id": "UNKNOWN:0003"
}